{
  "gene": "UniProtKB:Q13402",
  "gene_name": "Unconventional myosin-VIIa",
  "term_label": "actin filament organization",
  "gene_symbol": "MYO7A",
  "term_id": "GO:0007015"
}